{
  "gene_name": "Cyclin-dependent kinase 5 activator 1",
  "gene": "UniProtKB:Q15078",
  "gene_symbol": "CDK5R1",
  "term_id": "GO:0005737",
  "term_label": "cytoplasm"
}